{
  "gene": "UniProtKB:P08254",
  "gene_name": "Stromelysin-1",
  "term_id": "GO:0030574",
  "term_label": "collagen catabolic process",
  "gene_symbol": "MMP3"
}